{
  "gene": "UniProtKB:Q8IY95",
  "gene_name": "Transmembrane protein 192",
  "term_id": "GO:0005770",
  "gene_symbol": "TMEM192",
  "term_label": "late endosome"
}